{
  "term_label": "SNARE complex",
  "gene": "UniProtKB:Q13277",
  "gene_name": "Syntaxin-3",
  "term_id": "GO:0031201",
  "gene_symbol": "STX3"
}